response to pulsatile fluid shear stress [GO:0097701] (biological process) Definition: Any response to fluid shear stress where the fluid is flowing across a solid surface with periodic variations. For example, the endothelium in straight parts of the artery tree is subjected to pulsatile shear stress with a significant forward direction, which is believed to be an important physiological stimulus enhancing vessel compliance and conferring anti-thrombotic, anti-adhesive, and anti-inflammatory effects. References: PMID:21768538 Sources: GOC:BHF, GOC:BHF_miRNA, GOC:bc Relationships: is a type of GO:0034405 Subtypes: cellular response to pulsatile fluid shear stress [GO:0097703]